{
  "gene_symbol": "NPM1",
  "gene_name": "Nucleophosmin",
  "gene": "UniProtKB:P06748",
  "term_id": "GO:0005737",
  "term_label": "cytoplasm"
}